{
  "gene": "UniProtKB:Q1X8D7",
  "gene_name": "Leucine-rich repeat-containing protein 36",
  "gene_symbol": "LRRC36",
  "term_id": "UNKNOWN:0002",
  "term_label": "Unknown biological process"
}